{
  "gene_symbol": "ECSIT",
  "gene": "UniProtKB:Q9BQ95",
  "term_label": "cell surface receptor protein serine/threonine kinase signaling pathway",
  "term_id": "GO:0007178",
  "gene_name": "Evolutionarily conserved signaling intermediate in Toll pathway, mitochondrial"
}